{
  "gene": "UniProtKB:Q86WR0",
  "term_label": "Unknown biological process",
  "term_id": "UNKNOWN:0002",
  "gene_symbol": "CCDC25",
  "gene_name": "Coiled-coil domain-containing protein 25"
}